{
  "gene": "UniProtKB:Q6IQ22",
  "term_label": "plasma membrane",
  "gene_name": "Ras-related protein Rab-12",
  "term_id": "GO:0005886",
  "gene_symbol": "RAB12"
}